regulation of dopaminergic neuron differentiation [GO:1904338] (biological process) References: PMID:15522889 Sources: GOC:TermGenie, GO_REF:0000058 Definition: Any process that modulates the frequency, rate or extent of dopaminergic neuron differentiation. Relationships: is a type of regulation of neuron differentiation [GO:0045664]; regulates dopaminergic neuron differentiation [GO:0071542] Subtypes: negative regulation of dopaminergic neuron differentiation [GO:1904339], GO:1904340, GO:1904956